positive regulation of estrogen biosynthetic process [GO:1904078] (biological process) References: PMID:24530842 Sources: GOC:TermGenie, GO_REF:0000058 Relationships: is a type of positive regulation of steroid biosynthetic process [GO:0010893]; is a type of positive regulation of hormone biosynthetic process [GO:0046886]; is a type of GO:1904076; positively regulates estrogen biosynthetic process [GO:0006703] Also known as: positive regulation of estrogen anabolism, positive regulation of estrogen biosynthesis, positive regulation of estrogen formation, positive regulation of estrogen synthesis, positive regulation of oestrogen biosynthesis, positive regulation of oestrogen biosynthetic process, up regulation of estrogen anabolism, up regulation of estrogen biosynthesis, up regulation of estrogen biosynthetic process, up regulation of estrogen formation, up regulation of estrogen synthesis, up regulation of oestrogen biosynthesis, up regulation of oestrogen biosynthetic process, up-regulation of estrogen anabolism, up-regulation of estrogen biosynthesis, up-regulation of estrogen biosynthetic process, up-regulation of estrogen formation, up-regulation of estrogen synthesis, up-regulation of oestrogen biosynthesis, up-regulation of oestrogen biosynthetic process, upregulation of estrogen anabolism, upregulation of estrogen biosynthesis, upregulation of estrogen biosynthetic process, upregulation of estrogen formation, upregulation of estrogen synthesis, upregulation of oestrogen biosynthesis, upregulation of oestrogen biosynthetic process, activation of estrogen anabolism, activation of estrogen biosynthesis, activation of estrogen biosynthetic process, activation of estrogen formation, activation of estrogen synthesis, activation of oestrogen biosynthesis, activation of oestrogen biosynthetic process Definition: Any process that activates or increases the frequency, rate or extent of estrogen biosynthetic process.